{
  "term_id": "GO:0042806",
  "gene_symbol": "CLEC10A",
  "gene": "UniProtKB:Q8IUN9",
  "gene_name": "C-type lectin domain family 10 member A",
  "term_label": "fucose binding"
}